optomotor response [GO:0071632] (biological process) Definition: Eye, head or whole body movements that help to compensate movements of the environment in order to stabilize its image on the retina. In the case of whole body movements, these motor actions may also stabilize a locomotor course in response to some disturbance. Examples include: the optokinetic reflex, which allows human eyes to follow objects in motion while the head remains stationary reflex; the optomotor responses of flying insects and swimming fish. References: PMID:12726833, PMID:2469195 Sources: GOC:dos Relationships: is a type of optokinetic behavior [GO:0007634]